{
  "gene_symbol": "IDH1",
  "term_id": "GO:0006739",
  "gene_name": "Isocitrate dehydrogenase [NADP] cytoplasmic",
  "gene": "UniProtKB:O75874",
  "term_label": "NADP+ metabolic process"
}